{
  "gene_name": "Polypeptide N-acetylgalactosaminyltransferase 9",
  "term_id": "GO:0005794",
  "gene_symbol": "GALNT9",
  "gene": "UniProtKB:Q9HCQ5",
  "term_label": "Golgi apparatus"
}